{
  "gene": "UniProtKB:P00966",
  "term_label": "argininosuccinate synthase activity",
  "gene_name": "Argininosuccinate synthase",
  "gene_symbol": "ASS1",
  "term_id": "GO:0004055"
}